{
  "gene_symbol": "A0A8V8TII8",
  "term_id": "UNKNOWN:0001",
  "gene_name": "Uncharacterized protein",
  "term_label": "Unknown molecular function",
  "gene": "UniProtKB:A0A8V8TII8"
}